{
  "gene_name": "Immunoglobulin lambda variable 9-49",
  "term_label": "immunoglobulin complex",
  "gene_symbol": "IGLV9-49",
  "term_id": "GO:0019814",
  "gene": "UniProtKB:A0A0B4J1Y8"
}